juvenile hormone response element binding [GO:0070594] (molecular function) Also known as: JHRE binding Relationships: is a type of RNA polymerase II cis-regulatory region sequence-specific DNA binding [GO:0000978] References: PMID:17956872 Sources: GOC:sart Definition: Binding to a juvenile hormone response element (JHRE), a conserved sequence found in the promoters of genes whose expression is regulated in response to juvenile hormone.